{
  "term_id": "UNKNOWN:0002",
  "gene_symbol": "TSPAN8",
  "gene_name": "Tetraspanin-8",
  "term_label": "Unknown biological process",
  "gene": "UniProtKB:P19075"
}